negative regulation of hemopoiesis [GO:1903707] (biological process) Definition: Any process that stops, prevents or reduces the frequency, rate or extent of hemopoiesis. Subtypes: negative regulation of hematopoietic stem cell proliferation [GO:1902034], negative regulation of leukocyte differentiation [GO:1902106] Also known as: down regulation of blood cell biosynthesis, down regulation of blood cell formation, down regulation of haemopoiesis, down regulation of hematopoiesis, down regulation of hemopoiesis, down-regulation of blood cell biosynthesis, down-regulation of blood cell formation, down-regulation of haemopoiesis, down-regulation of hematopoiesis, down-regulation of hemopoiesis, downregulation of blood cell biosynthesis, downregulation of blood cell formation, downregulation of haemopoiesis, downregulation of hematopoiesis, downregulation of hemopoiesis, negative regulation of blood cell biosynthesis, negative regulation of blood cell formation, negative regulation of haemopoiesis, negative regulation of hematopoiesis, inhibition of blood cell biosynthesis, inhibition of blood cell formation, inhibition of haemopoiesis, inhibition of hematopoiesis, inhibition of hemopoiesis Relationships: is a type of negative regulation of immune system process [GO:0002683]; is a type of negative regulation of cell development [GO:0010721]; is a type of GO:0051241; is a type of regulation of hemopoiesis [GO:1903706]; negatively regulates hemopoiesis [GO:0030097] References: PMID:20080761 Sources: GOC:PARL, GOC:TermGenie, GOC:pad, GO_REF:0000058 Note: An example of this is Atg7 in mouse (UniProt symbol, Q9D906) in PMID:20080761, inferred from mutant phenotype.